protein localization to myelin sheath abaxonal region [GO:0035750] (biological process) References: PMID:20237282 Sources: GOC:BHF Also known as: protein localisation to myelin sheath abaxonal region Relationships: is a type of intracellular protein localization [GO:0008104] Definition: Any process in which a protein is transported to, and/or maintained in, the abaxonal region of the myelin sheath. The abaxonal region is the region of the myelin sheath furthest from the axon.